post-embryonic camera-type eye development [GO:0031077] (biological process) Also known as: post-embryonic camera-style eye development Sources: GOC:mah, GOC:mtg_sensu Definition: The process occurring during the post-embryonic phase whose specific outcome is the progression of the camera-type eye over time, from its formation to the mature structure. Relationships: is a type of camera-type eye development [GO:0043010]; is part of post-embryonic development [GO:0009791]